negative regulation of G1/S transition of mitotic cell cycle [GO:2000134] (biological process) Sources: GOC:mtg_cell_cycle Definition: Any signaling pathway that decreases or inhibits the activity of a cell cycle cyclin-dependent protein kinase to modulate the switch from G1 phase to S phase of the mitotic cell cycle. Relationships: is a type of GO:1901991; is a type of GO:1902807; is a type of GO:2000045; negatively regulates GO:0000082 Subtypes: mitotic G1 cell size control checkpoint signaling [GO:0031568], mitotic G1/S transition checkpoint signaling [GO:0044819]